{
  "gene_symbol": "COL5A1",
  "gene_name": "Collagen alpha-1(V) chain",
  "term_label": "extracellular matrix",
  "gene": "UniProtKB:P20908",
  "term_id": "GO:0031012"
}